{
  "gene": "UniProtKB:Q96BD0",
  "term_label": "basolateral plasma membrane",
  "gene_symbol": "SLCO4A1",
  "term_id": "GO:0016323",
  "gene_name": "Solute carrier organic anion transporter family member 4A1"
}